{
  "term_id": "GO:0032933",
  "term_label": "SREBP signaling pathway",
  "gene_symbol": "INSIG2",
  "gene": "UniProtKB:Q9Y5U4",
  "gene_name": "Insulin-induced gene 2 protein"
}